{
  "gene": "UniProtKB:Q8N112",
  "term_id": "UNKNOWN:0003",
  "term_label": "Unknown cellular component",
  "gene_symbol": "LSMEM2",
  "gene_name": "Leucine-rich single-pass membrane protein 2"
}